mithramycin dehydrogenase (NADPH) activity [GO:0102357] (MF) Definition: Catalysis of the reaction: mithramycin DK + NADPH + H+ = iso-mithramycin + NADP+. Note that  iso-mithramycin (iso-MTM) is a C2-epimer of mithramycin.  This intermediate appears to be biologically important because it is non-toxic, then exported out of the cell and finally spontaneously epimerized into the toxic mithramycin. This could represent a self-resistance mechanism against MTM toxicity. Relationships: is_a GO:0016616 References: PMID:31702856